{
  "term_label": "plasma membrane",
  "gene_symbol": "NPY4R",
  "term_id": "GO:0005886",
  "gene_name": "Neuropeptide Y receptor type 4",
  "gene": "UniProtKB:P50391"
}